{
  "term_label": "cellular response to lipopolysaccharide",
  "gene_name": "C-X-C motif chemokine 13",
  "gene_symbol": "CXCL13",
  "term_id": "GO:0071222",
  "gene": "UniProtKB:O43927"
}